{
  "term_label": "Unknown cellular component",
  "gene": "UniProtKB:Q8NA70",
  "gene_symbol": "FAM47B",
  "gene_name": "Protein FAM47B",
  "term_id": "UNKNOWN:0003"
}